primary cell septum disassembly [GO:0030994] (biological process) References: PMID:12665550 Definition: Dissolution of the primary septum during cell separation. Also known as: primary septum hydrolysis, hydrolysis of primary cell septum, primary cell septum hydrolysis Relationships: is a type of cellular component disassembly [GO:0022411]; is part of septum digestion after cytokinesis [GO:0000920]